{
  "gene_name": "E3 ubiquitin-protein ligase TRIM69",
  "gene_symbol": "TRIM69",
  "gene": "UniProtKB:Q86WT6",
  "term_label": "ubiquitin protein ligase activity",
  "term_id": "GO:0061630"
}